{
  "gene_symbol": "HLA-A",
  "gene": "UniProtKB:P04439",
  "gene_name": "HLA class I histocompatibility antigen, A alpha chain",
  "term_label": "peptide antigen binding",
  "term_id": "GO:0042605"
}